protein secretion by platelet [GO:0070560] (biological process) Relationships: is a type of protein secretion [GO:0009306]; is a type of establishment of localization in cell [GO:0051649]; is a type of exocytic process [GO:0140029]; is part of platelet degranulation [GO:0002576] Definition: The regulated release of proteins by a platelet or group of platelets. Sources: GOC:BHF, GOC:mah